regulatory ncRNA-mediated post-transcriptional gene silencing [GO:0035194] (biological process) References: PMID:11201747, PMID:11713190, PMID:15020054, PMID:15066275, PMID:18771919, PMID:32885814, PMID:33184244 Sources: GOC:ems Definition: A posttranscriptional gene silencing pathway in which regulatory RNAs elicit silencing of specific target genes, either by mRNA destabilization or inhibition of translation. Relationships: is a type of post-transcriptional gene silencing [GO:0016441]; is a type of GO:0031047 Regulation: regulated by regulation of post-transcriptional gene silencing by regulatory ncRNA [GO:1900368]; negatively regulated by negative regulation of post-transcriptional gene silencing by regulatory ncRNA [GO:1900369]; positively regulated by positive regulation of post-transcriptional gene silencing by RNA [GO:1900370] Subtypes: lncRNA-mediated post-transcriptional gene silencing [GO:0000512], GO:0009616, miRNA-mediated post-transcriptional gene silencing [GO:0035195], transitive RNA interference [GO:0036453], sRNA-mediated post-transcriptional gene silencing [GO:0040033], siRNA-mediated post-transcriptional gene silencing [GO:0140766], GO:0140991 Also known as: PTGS, RNA interference, RNAi, RNA-dependent post-transcriptional gene silencing, RNA-mediated post-transcriptional gene silencing, RNA-mediated posttranscriptional gene silencing, ncRNA-mediated post-transcriptional gene silencing, posttranscriptional gene silencing by RNA, cosuppression, post-transcriptional gene silencing by RNA, quelling